negative regulation of mitotic actomyosin contractile ring assembly [GO:1903500] (biological process) Subtypes: negative regulation of protein localization to cell division site involved in mitotic actomyosin contractile ring assembly [GO:0110084] References: PMID:18256290 Sources: GOC:TermGenie, GOC:al, GOC:mtg_cell_cycle, GOC:vw, GO_REF:0000058 Definition: Any process that stops, prevents or reduces the frequency, rate or extent of mitotic actomyosin contractile ring assembly. Relationships: is a type of negative regulation of mitotic cytokinetic process [GO:1903437]; is a type of regulation of mitotic actomyosin contractile ring assembly [GO:1903499]; is a type of GO:2000432; negatively regulates GO:1903475 Also known as: down regulation of actomyosin contractile ring assembly involved in cytokinesis after mitosis, down regulation of contractile ring assembly involved in mitotic cytokinesis, down regulation of cytokinesis, actomyosin contractile ring assembly involved in mitotic cytokinesis, down regulation of mitotic actomyosin contractile ring assembly, down-regulation of actomyosin contractile ring assembly involved in cytokinesis after mitosis, down-regulation of contractile ring assembly involved in mitotic cytokinesis, down-regulation of cytokinesis, actomyosin contractile ring assembly involved in mitotic cytokinesis, down-regulation of mitotic actomyosin contractile ring assembly, downregulation of actomyosin contractile ring assembly involved in cytokinesis after mitosis, downregulation of contractile ring assembly involved in mitotic cytokinesis, downregulation of cytokinesis, actomyosin contractile ring assembly involved in mitotic cytokinesis, downregulation of mitotic actomyosin contractile ring assembly, negative regulation of actomyosin contractile ring assembly involved in cytokinesis after mitosis, negative regulation of contractile ring assembly involved in mitotic cytokinesis, negative regulation of cytokinesis, actomyosin contractile ring assembly involved in mitotic cytokinesis, negative regulation of mitotic cytokinesis, actomyosin contractile ring assembly, inhibition of actomyosin contractile ring assembly involved in cytokinesis after mitosis, inhibition of contractile ring assembly involved in mitotic cytokinesis, inhibition of cytokinesis, actomyosin contractile ring assembly involved in mitotic cytokinesis, inhibition of mitotic actomyosin contractile ring assembly